aortic valve development [GO:0003176] (biological process) Sources: GOC:mtg_heart Definition: The progression of the aortic valve over time, from its formation to the mature structure. Relationships: is a type of GO:1905314